{
  "gene_symbol": "PNLIPRP2",
  "gene": "UniProtKB:P54317",
  "term_label": "triglyceride catabolic process",
  "gene_name": "Pancreatic lipase-related protein 2",
  "term_id": "GO:0019433"
}